{
  "term_id": "GO:0006457",
  "gene_symbol": "PFDN1",
  "gene_name": "Prefoldin subunit 1",
  "gene": "UniProtKB:O60925",
  "term_label": "protein folding"
}